{
  "gene_symbol": "TTC33",
  "term_id": "UNKNOWN:0002",
  "gene_name": "Tetratricopeptide repeat protein 33",
  "term_label": "Unknown biological process",
  "gene": "UniProtKB:Q6PID6"
}